vitamin transmembrane transporter activity [GO:0090482] (molecular function) Also known as: vitamin or cofactor transporter activity, vitamin transporter activity Sources: GOC:tb Definition: Enables the transfer of a vitamin from one side of a membrane to the other. Relationships: is_a transmembrane transporter activity [GO:0022857]; is part of vitamin transmembrane transport [GO:0035461] Subtypes: folic acid transmembrane transporter activity [GO:0008517], sodium-dependent multivitamin transmembrane transporter activity [GO:0008523], biotin transmembrane transporter activity [GO:0015225], L-ascorbic acid transmembrane transporter activity [GO:0015229], pantothenate transmembrane transporter activity [GO:0015233], thiamine transmembrane transporter activity [GO:0015234], ABC-type vitamin B12 transporter activity [GO:0015420], GO:0031924, riboflavin transmembrane transporter activity [GO:0032217], GO:0033300, retinol transmembrane transporter activity [GO:0034632]